{
  "term_id": "GO:0004801",
  "gene_name": "Transaldolase",
  "gene_symbol": "TALDO1",
  "term_label": "transaldolase activity",
  "gene": "UniProtKB:P37837"
}